cortical collecting duct development [GO:0072059] (biological process) Definition: The process whose specific outcome is the progression of the cortical collecting duct over time, from its formation to the mature structure. The cortical collecting duct is the portion of the collecting duct that resides in the renal cortex. Sources: GOC:mtg_kidney_jan10 Relationships: is a type of GO:0048856 Subtypes: GO:0072219